positive regulation of eukaryotic translation initiation factor 4F complex assembly [GO:1905537] (biological process) Definition: Any process that activates or increases the frequency, rate or extent of eukaryotic translation initiation factor 4F complex assembly. References: PMID:18426977 Sources: GOC:PARL, GOC:TermGenie, GOC:bc, GO_REF:0000058 Also known as: positive regulation of eIF-4F assembly, positive regulation of eIF4F assembly, up regulation of eIF-4F assembly, up regulation of eIF4F assembly, up regulation of eukaryotic translation initiation factor 4F complex assembly, up-regulation of eIF-4F assembly, up-regulation of eIF4F assembly, up-regulation of eukaryotic translation initiation factor 4F complex assembly, upregulation of eIF-4F assembly, upregulation of eIF4F assembly, upregulation of eukaryotic translation initiation factor 4F complex assembly, activation of eIF-4F assembly, activation of eIF4F assembly, activation of eukaryotic translation initiation factor 4F complex assembly Relationships: is a type of positive regulation of protein-containing complex assembly [GO:0031334]; is a type of GO:1905535; positively regulates eukaryotic translation initiation factor 4F complex assembly [GO:0097010]